L-seryl-tRNA(Sec) selenium transferase activity [GO:0004125] (molecular function) Definition: Catalysis of the reaction: L-seryl-tRNA(Sec) + selenophosphate = L-selenocysteinyl-tRNA(Sec) + H2O + phosphate. Relationships: is a type of selenotransferase activity [GO:0016785]; is a type of catalytic activity, acting on a tRNA [GO:0140101] Sources: RHEA:22728 Also known as: L-seryl-tRNASec selenium transferase activity, cysteinyl-tRNA(Ser) selenium transferase activity, selenocysteine synthase activity, selenocysteinyl-tRNA(Ser) synthase activity, L-selenocysteinyl-tRNA(Sec) synthase activity, L-selenocysteinyl-tRNA(Sel) synthase activity, L-selenocysteinyl-tRNASec synthase activity, L-selenocysteinyl-tRNASel synthase activity, cysteinyl-tRNA(Sec)-selenium transferase activity, cysteinyl-tRNA(Sel)-selenium transferase activity, cysteinyl-tRNASec-selenium transferase activity, cysteinyl-tRNASel-selenium transferase activity, selenophosphate:L-seryl-tRNASec selenium transferase activity